{
  "term_label": "cytoplasm",
  "gene_symbol": "RNPS1",
  "gene": "UniProtKB:Q15287",
  "gene_name": "RNA-binding protein with serine-rich domain 1",
  "term_id": "GO:0005737"
}